{
  "term_id": "GO:0005794",
  "gene": "UniProtKB:Q5M8T2",
  "gene_name": "Solute carrier family 35 member D3",
  "term_label": "Golgi apparatus",
  "gene_symbol": "SLC35D3"
}